defecation [GO:0030421] (biological process) Sources: GOC:mah Definition: The expulsion of feces from the rectum. Relationships: is a type of excretion [GO:0007588]; is a type of digestive system process [GO:0022600] Regulation: regulated by regulation of defecation [GO:2000292]; RO_0002212 by negative regulation of defecation [GO:2000293]; RO_0002213 by positive regulation of defecation [GO:2000294]